hydro-lyase activity [GO:0016836] (molecular function) Sources: EC:4.2.1.- Subtypes: GO:0003855, 3-isopropylmalate dehydratase activity [GO:0003861], aconitate hydratase activity [GO:0003994], GO:0004089, GO:0004122, dihydroxy-acid dehydratase activity [GO:0004160], GO:0004300, fumarate hydratase activity [GO:0004333], homoaconitate hydratase activity [GO:0004409], imidazoleglycerol-phosphate dehydratase activity [GO:0004424], phosphogluconate dehydratase activity [GO:0004456], methylglutaconyl-CoA hydratase activity [GO:0004490], phosphopyruvate hydratase activity [GO:0004634], porphobilinogen synthase activity [GO:0004655], prephenate dehydratase activity [GO:0004664], pseudouridylate synthase activity [GO:0004730], tryptophan synthase activity [GO:0004834], uroporphyrinogen-III synthase activity [GO:0004852], 4-alpha-hydroxytetrahydrobiopterin dehydratase activity [GO:0008124], GDP-mannose 4,6-dehydratase activity [GO:0008446], GO:0008460, GO:0008684, L(+)-tartrate dehydratase activity [GO:0008730], altronate dehydratase activity [GO:0008789], 4-hydroxy-tetrahydrodipicolinate synthase activity [GO:0008840], galactarate dehydratase activity [GO:0008867], GO:0008869, glucarate dehydratase activity [GO:0008872], GO:0008927, allene oxide synthase activity [GO:0009978], urocanate hydratase activity [GO:0016153], retinol dehydratase activity [GO:0017051], cyclohex-1-ene-1-carboxyl-CoA hydratase activity [GO:0018811], trans-o-hydroxybenzylidenepyruvate hydratase-aldolase activity [GO:0018813], 3-methyl-5-hydroxy-6-(3-carboxy-3-oxopropenyl)-1H-2-pyridon hydratase-aldolase activity [GO:0018815], GO:0018817, GO:0018818, lactoyl-CoA dehydratase activity [GO:0018819], cyanamide hydratase activity [GO:0018820], nitrile hydratase activity [GO:0018822], cyclohexa-1,5-dienecarbonyl-CoA hydratase activity [GO:0018823], (3R)-hydroxyacyl-[acyl-carrier-protein] dehydratase activity [GO:0019171], glyoxalase III activity [GO:0019172], cyanide hydratase activity [GO:0030196], scytalone dehydratase activity [GO:0030411], 2-hydroxyisoflavanone dehydratase activity [GO:0033987], GO:0033988, 3alpha,7alpha,12alpha-trihydroxy-5beta-cholest-24-enoyl-CoA hydratase activity [GO:0033989], ectoine synthase activity [GO:0033990], GO:0033991, GO:0033992, 2-hydroxyhexa-2,4-dienoate hydratase activity [GO:0034856], 2-hydroxyglutaryl-CoA dehydratase activity [GO:0043717], 4-hydroxybutanoyl-CoA dehydratase activity [GO:0043721], 2-keto-3-deoxygalactonate aldolase activity [GO:0043724], O-succinylbenzoate synthase activity [GO:0043748], mesaconyl-CoA hydratase activity [GO:0043881], L-erythro-3-methylmalyl-CoA dehydratase activity [GO:0043960], glycerol dehydratase activity [GO:0046405], GO:0046565, GO:0046570, 5-dehydro-4-deoxyglucarate dehydratase activity [GO:0047448], 2-dehydro-3-deoxy-L-arabinonate dehydratase activity [GO:0047449], protoaphin-aglucone dehydratase (cyclizing) activity [GO:0047452], GO:0047453, phaseollidin hydratase activity [GO:0047454], GO:0047455, GO:0047456, GO:0047508, (S)-2-methylmalate dehydratase activity [GO:0047510], GO:0047547, 3-cyanoalanine hydratase activity [GO:0047558], GO:0047584, 5-alpha-hydroxysteroid dehydratase activity [GO:0047587], arabinonate dehydratase activity [GO:0047675], CDP-glucose 4,6-dehydratase activity [GO:0047733], arogenate dehydratase activity [GO:0047769], D(-)-tartrate dehydratase activity [GO:0047808], D-fuconate dehydratase activity [GO:0047818], GO:0047820, GO:0047868, gluconate dehydratase activity [GO:0047929], isohexenylglutaconyl-CoA hydratase activity [GO:0050005], itaconyl-CoA hydratase activity [GO:0050011], kievitone hydratase activity [GO:0050015], GO:0050020, GO:0050023, L-rhamnonate dehydratase activity [GO:0050032], maleate hydratase activity [GO:0050075], acetylenecarboxylate hydratase activity [GO:0050079], myo-inosose-2 dehydratase activity [GO:0050114], oleate hydratase activity [GO:0050151], octopamine dehydratase activity [GO:0050202], propanediol dehydratase activity [GO:0050215], pyrazolylalanine synthase activity [GO:0050234], GO:0050315, trans-L-3-hydroxyproline dehydratase activity [GO:0050346], UDP-glucose 4,6-dehydratase activity [GO:0050377], xylonate dehydratase activity [GO:0050401], cyclohexyl-isocyanide hydratase activity [GO:0050549], L-serine hydro-lyase (adding indole, L-tryptophan-forming) activity [GO:0052684], ADP-dependent NAD(P)H-hydrate dehydratase activity [GO:0052855], tRNA threonylcarbamoyladenosine dehydratase [GO:0061503], 6-carboxytetrahydropterin synthase activity [GO:0070497], GO:0098605, copal-8-ol diphosphate synthase activity [GO:0102161], lupan-3beta,20-diol synthase activity [GO:0102245], pterin-4alpha-carbinolamine dehydratase activity [GO:0102434], 17(E)-cheilanthenediol synthase activity [GO:0102645], 14betaH-scalarane-17alpha-19-diol synthase activity [GO:0102646], GO:0102895, peregrinol diphosphate synthase activity [GO:0106238], hydroperoxy icosatetraenoate dehydratase activity [GO:0106256], 2-(omega-methylthio)alkylmalate dehydratase activity [GO:0120528], pterocarpan synthase activity [GO:0140859], glyoxalase (glycolic acid-forming) activity [GO:1990422], GO:1990594 Relationships: is a type of carbon-oxygen lyase activity [GO:0016835] Definition: Catalysis of the cleavage of a carbon-oxygen bond by elimination of water.